{
  "term_id": "GO:0005829",
  "gene_symbol": "DCTPP1",
  "gene_name": "dCTP pyrophosphatase 1",
  "gene": "UniProtKB:Q9H773",
  "term_label": "cytosol"
}